{
  "gene_symbol": "RNF2",
  "term_label": "PcG protein complex",
  "gene_name": "E3 ubiquitin-protein ligase RING2",
  "gene": "UniProtKB:Q99496",
  "term_id": "GO:0031519"
}